glycogen granule [GO:0042587] (CC) References: PMID:12179957 Sources: GOC:jl Definition: Cytoplasmic bead-like structures of animal cells, visible by electron microscope. Each granule is a functional unit with the biosynthesis and catabolism of glycogen being catalyzed by enzymes bound to the granule surface. Also known as: glycogen particle Relationships: is a type of cellular anatomical structure [GO:0110165]; is part of cytoplasm [GO:0005737]